{
  "gene": "UniProtKB:Q9Y2S2",
  "gene_name": "Lambda-crystallin homolog",
  "term_label": "Unknown cellular component",
  "gene_symbol": "CRYL1",
  "term_id": "UNKNOWN:0003"
}